{
  "gene": "UniProtKB:Q15303",
  "gene_symbol": "ERBB4",
  "gene_name": "Receptor tyrosine-protein kinase erbB-4",
  "term_label": "epidermal growth factor receptor signaling pathway",
  "term_id": "GO:0007173"
}